{
  "gene_symbol": "IGHV3OR16-8",
  "gene": "UniProtKB:A0A075B7F1",
  "gene_name": "Immunoglobulin heavy variable 3_OR16-8 (non-functional) (Fragment)",
  "term_label": "immunoglobulin mediated immune response",
  "term_id": "GO:0016064"
}